{
  "gene": "UniProtKB:Q7Z5A7",
  "gene_name": "Chemokine-like protein TAFA-5",
  "term_id": "GO:0007186",
  "term_label": "G protein-coupled receptor signaling pathway",
  "gene_symbol": "TAFA5"
}